{
  "gene_name": "Uncharacterized protein C19orf44",
  "term_id": "UNKNOWN:0003",
  "term_label": "Unknown cellular component",
  "gene": "UniProtKB:Q9H6X5",
  "gene_symbol": "C19orf44"
}